{
  "gene": "UniProtKB:Q01813",
  "term_label": "membrane",
  "gene_name": "ATP-dependent 6-phosphofructokinase, platelet type",
  "gene_symbol": "PFKP",
  "term_id": "GO:0016020"
}